lovastatin nonaketide synthase activity [GO:0050637] (molecular function) Definition: Catalysis of the reaction: S-adenosyl-L-methionine(1+) + acetyl-CoA + 18 H+ + 8 malonyl-CoA + 11 NADPH = S-adenosyl-L-homocysteine + 8 CO2 + 9 CoA + dihydromonacolin L + 6 H2O + 11 NADP+. Sources: EC:2.3.1.161, RHEA:18565 Also known as: acyl-CoA:malonyl-CoA C-acyltransferase (decarboxylating, oxoacyl- and enoyl-reducing, thioester-hydrolysing) Relationships: is a type of GO:0016747